{
  "gene_name": "Neuronal acetylcholine receptor subunit alpha-7",
  "term_id": "GO:0034220",
  "gene_symbol": "CHRNA7",
  "term_label": "monoatomic ion transmembrane transport",
  "gene": "UniProtKB:P36544"
}